{
  "gene_symbol": "HID1",
  "term_label": "Unknown biological process",
  "gene_name": "Protein HID1",
  "term_id": "UNKNOWN:0002",
  "gene": "UniProtKB:Q8IV36"
}